{
  "term_id": "GO:0006400",
  "gene_name": "tRNA dimethylallyltransferase",
  "term_label": "tRNA modification",
  "gene_symbol": "TRIT1",
  "gene": "UniProtKB:Q9H3H1"
}